dsRNA transport [GO:0033227] (biological process) Definition: The directed movement of dsRNA, double-stranded ribonucleic acid, into, out of or within a cell, or between cells, by means of some agent such as a transporter or pore. Sources: GOC:mah Relationships: is a type of RNA transport [GO:0050658]